Delta24-sterol reductase activity [GO:0050614] (molecular function) Sources: EC:1.3.1.72 Also known as: D24-sterol reductase activity, lanosterol Delta(24)-reductase activity, lanosterol delta24-reductase activity, sterol:NADP+ delta24-oxidoreductase activity Definition: Catalysis of the reaction: NADP+ + 5-alpha-cholest-7-en-3-beta-ol = NADPH + H+ + 5-alpha-cholesta-7,24-dien-3-beta-ol. Relationships: is a type of GO:0016628